{
  "gene": "UniProtKB:O94829",
  "term_label": "protein import into nucleus",
  "term_id": "GO:0006606",
  "gene_name": "Importin-13",
  "gene_symbol": "IPO13"
}